{
  "term_id": "GO:0000981",
  "term_label": "DNA-binding transcription factor activity, RNA polymerase II-specific",
  "gene": "UniProtKB:O60675",
  "gene_name": "Transcription factor MafK",
  "gene_symbol": "MAFK"
}